{
  "gene": "UniProtKB:O75354",
  "gene_symbol": "ENTPD6",
  "term_label": "Golgi apparatus",
  "term_id": "GO:0005794",
  "gene_name": "Ectonucleoside triphosphate diphosphohydrolase 6"
}